negative regulation of anterior neural cell fate commitment of the neural plate [GO:0022001] (biological process) Definition: Any process that stops, prevents or reduces the frequency or rate at which a cell adopts an anterior neural cell fate. Subtypes: GO:0022003 Relationships: is a type of GO:0010454; is a type of negative regulation of nervous system development [GO:0051961]; is part of neural plate anterior/posterior regionalization [GO:0021999] Also known as: posteriorization, caudalization of neural plate, down regulation of anterior neural cell fate of the neural plate, down-regulation of anterior neural cell fate of the neural plate, downregulation of anterior neural cell fate of the neural plate, negative regulation of anterior neural cell fate of the neural plate, inhibition of anterior neural cell fate of the neural plate Sources: GOC:cls, GOC:dgh, GOC:dph, GOC:jid, GOC:tb